{
  "term_id": "GO:0008154",
  "gene_name": "Villin-like protein",
  "term_label": "actin polymerization or depolymerization",
  "gene_symbol": "VILL",
  "gene": "UniProtKB:O15195"
}